{
  "gene": "UniProtKB:O14975",
  "gene_symbol": "SLC27A2",
  "term_id": "GO:0004467",
  "term_label": "long-chain fatty acid-CoA ligase activity",
  "gene_name": "Long-chain fatty acid transport protein 2"
}